{
  "term_id": "UNKNOWN:0002",
  "gene_symbol": "SNRNP27",
  "gene_name": "U4_U6.U5 small nuclear ribonucleoprotein 27 kDa protein",
  "gene": "UniProtKB:Q8WVK2",
  "term_label": "Unknown biological process"
}